{
  "gene": "UniProtKB:Q9NQG7",
  "gene_symbol": "HPS4",
  "gene_name": "BLOC-3 complex member HPS4",
  "term_label": "protein targeting",
  "term_id": "GO:0006605"
}